{
  "term_id": "GO:0005745",
  "gene_name": "AFG3-like protein 2",
  "gene_symbol": "AFG3L2",
  "term_label": "m-AAA complex",
  "gene": "UniProtKB:Q9Y4W6"
}